{
  "gene": "UniProtKB:Q6X4W1",
  "gene_name": "NMDA receptor synaptonuclear signaling and neuronal migration factor",
  "term_id": "GO:0005737",
  "term_label": "cytoplasm",
  "gene_symbol": "NSMF"
}